nitrite reductase (cytochrome, ammonia-forming) activity [GO:0042279] (MF) Also known as: cytochrome c nitrite reductase activity, multiheme nitrite reductase activity, cytochrome c552 activity, ammonia:ferricytochrome-c oxidoreductase activity, nitrite reductase (cytochrome; ammonia-forming) Relationships: is a type of oxidoreductase activity, acting on other nitrogenous compounds as donors, cytochrome as acceptor [GO:0016662]; is a type of nitrite reductase activity [GO:0098809] Definition: Catalysis of the reaction: 6 Fe(III)-[cytochrome c] + NH4+ + 2 H2O = 6 Fe(II)-[cytochrome c] + nitrite + 8 H+. Sources: RHEA:13089